{
  "gene": "UniProtKB:Q9UKL2",
  "gene_symbol": "OR52A1",
  "term_label": "olfactory receptor activity",
  "gene_name": "Olfactory receptor 52A1",
  "term_id": "GO:0004984"
}